alkali metal ion binding [GO:0031420] (molecular function) Definition: Binding to an alkali metal ion; alkali metals are those elements in group Ia of the periodic table, with the exception of hydrogen. Subtypes: potassium ion binding [GO:0030955], sodium ion binding [GO:0031402], lithium ion binding [GO:0031403] Relationships: is a type of metal ion binding [GO:0046872] Sources: GOC:mah